metabolic process [GO:0008152] (biological process) Sources: GOC:go_curators, ISBN:0198547684 Also known as: metabolism Regulation: negatively regulated by negative regulation of metabolic process [GO:0009892]; positively regulated by GO:0009893; regulated by regulation of metabolic process [GO:0019222]; negatively regulated by catabolite repression [GO:0061984] Note: Note that metabolic processes do not include single functions or processes such as protein-protein interactions, protein-nucleic acids, nor receptor-ligand interactions. Subtypes: GO:0001887, GO:0006081, generation of precursor metabolites and energy [GO:0006091], translational initiation [GO:0006413], peptide metabolic process [GO:0006518], modified amino acid metabolic process [GO:0006575], sulfur compound metabolic process [GO:0006790], phosphorus metabolic process [GO:0006793], xenobiotic metabolic process [GO:0006805], bioluminescence [GO:0008218], GO:0008291, catabolic process [GO:0009056], GO:0009058, GO:0009308, flavonoid metabolic process [GO:0009812], GO:0009820, carbon fixation [GO:0015977], GO:0015979, GO:0016999, nicotine metabolic process [GO:0018933], GO:0018942, phenol-containing compound metabolic process [GO:0018958], aldoxime metabolic process [GO:0019330], cyanide metabolic process [GO:0019499], GO:0019695, secondary metabolic process [GO:0019748], methylation [GO:0032259], collagen metabolic process [GO:0032963], tetrapyrrole metabolic process [GO:0033013], ketone metabolic process [GO:0042180], GO:0042360, indole-containing compound metabolic process [GO:0042430], GO:0042440, hormone metabolic process [GO:0042445], benzene-containing compound metabolic process [GO:0042537], GO:0042558, poly(3-hydroxyalkanoate) metabolic process [GO:0042620], flavin-containing compound metabolic process [GO:0042726], macromolecule metabolic process [GO:0043170], GO:0043603, primary metabolic process [GO:0044238], small molecule metabolic process [GO:0044281], GO:0045730, nitrile metabolic process [GO:0050898], prosthetic group metabolic process [GO:0051189], imidazole-containing compound metabolic process [GO:0052803], chemosynthesis [GO:0062097], demethylation [GO:0070988], nitrogen cycle metabolic process [GO:0071941], purine-containing compound metabolic process [GO:0072521], GO:0072524, pyrimidine-containing compound metabolic process [GO:0072527], oxygen metabolic process [GO:0072592], GO:0072593, organohalogen metabolic process [GO:0090345], epoxide metabolic process [GO:0097176], prenylation [GO:0097354], metabolite repair [GO:0110051], GO:0120252, olefinic compound metabolic process [GO:0120254], futile creatine cycle [GO:0140651], methanophenazine metabolic process [GO:1900629], carbohydrate derivative metabolic process [GO:1901135], GO:1901275, GO:1901286, lactone metabolic process [GO:1901334], GO:1901440, phosphinothricin metabolic process [GO:1901764], hydrogen metabolic process [GO:1902421], adaptive thermogenesis [GO:1990845], reactive nitrogen species metabolic process [GO:2001057], methanofuran metabolic process [GO:2001119] Definition: A cellular process consisting of the biochemical pathways by which a living organism transforms chemical substances. This includes including anabolism (biosynthetic process) and catabolism (catabolic process). Metabolic processes includes the transformation of small molecules, as well  macromolecular processes such as DNA repair and replication, protein synthesis and degradation. Relationships: is a type of cellular process [GO:0009987]